{
  "term_id": "GO:0001845",
  "gene_name": "Sushi repeat-containing protein SRPX",
  "term_label": "phagolysosome assembly",
  "gene": "UniProtKB:P78539",
  "gene_symbol": "SRPX"
}